N-terminal protein myristoylation [GO:0006499] (biological process) Relationships: is a type of N-terminal protein lipidation [GO:0006498]; is_a protein myristoylation [GO:0018377] Subtypes: GO:0018008 Sources: GOC:mah Definition: The covalent attachment of a myristoyl group to the N-terminal amino acid residue of a protein.